{
  "term_id": "UNKNOWN:0001",
  "gene": "UniProtKB:Q52LC2",
  "gene_symbol": "ATP6AP1L",
  "term_label": "Unknown molecular function",
  "gene_name": "V-type proton ATPase subunit S1-like protein"
}